{
  "gene": "UniProtKB:Q8NE35",
  "term_id": "GO:0150052",
  "gene_symbol": "CPEB3",
  "gene_name": "Cytoplasmic polyadenylation element-binding protein 3",
  "term_label": "regulation of postsynapse assembly"
}